amylin receptor complex 2 [GO:0150057] (cellular component) Definition: A G protein-coupled receptor complex that serves as a receptor for amylin polypeptide (AMY) and consists of a calcitonin receptor (CTR/CALCR) and a receptor activity-modifying protein (RAMP) 2. Amylin receptor complex 2 (AMY2) also serves as a receptor for adrenomedullin (AM/ADM). Also known as: AMY2 complex Relationships: is a type of amylin receptor complex [GO:1903440] References: PMID:22500019 Sources: GOC:aruk, GOC:bc